{
  "gene": "UniProtKB:Q8TDW0",
  "term_id": "GO:0034702",
  "term_label": "monoatomic ion channel complex",
  "gene_symbol": "LRRC8C",
  "gene_name": "Volume-regulated anion channel subunit LRRC8C"
}